{
  "gene_symbol": "ADAMTS7",
  "term_id": "GO:0031012",
  "gene": "UniProtKB:Q9UKP4",
  "term_label": "extracellular matrix",
  "gene_name": "A disintegrin and metalloproteinase with thrombospondin motifs 7"
}